{
  "term_id": "GO:0007409",
  "gene_symbol": "CDHR2",
  "term_label": "axonogenesis",
  "gene": "UniProtKB:Q9BYE9",
  "gene_name": "Cadherin-related family member 2"
}